{
  "term_label": "protein folding",
  "term_id": "GO:0006457",
  "gene_name": "Hsp90 co-chaperone Cdc37-like 1",
  "gene_symbol": "CDC37L1",
  "gene": "UniProtKB:Q7L3B6"
}